regulation of octopamine signaling pathway [GO:2000128] (biological process) Subtypes: negative regulation of octopamine signaling pathway [GO:2000129], positive regulation of octopamine signaling pathway [GO:2000130], regulation of octopamine signaling pathway involved in response to food [GO:2000139] Definition: Any process that modulates the frequency, rate or extent of octopamine signaling pathway. Sources: GOC:mah Also known as: regulation of octopamine signalling pathway Relationships: is_a regulation of octopamine or tyramine signaling pathway [GO:2000125]; regulates GO:0071927